{
  "term_id": "GO:0035313",
  "gene": "UniProtKB:Q8N264",
  "gene_symbol": "ARHGAP24",
  "gene_name": "Rho GTPase-activating protein 24",
  "term_label": "wound healing, spreading of epidermal cells"
}